{
  "gene_symbol": "AP1G2",
  "gene": "UniProtKB:O75843",
  "term_label": "clathrin adaptor activity",
  "term_id": "GO:0035615",
  "gene_name": "AP-1 complex subunit gamma-like 2"
}